{
  "gene_symbol": "TSC2",
  "gene": "UniProtKB:P49815",
  "term_label": "negative regulation of phosphatidylinositol 3-kinase/protein kinase B signal transduction",
  "term_id": "GO:0051898",
  "gene_name": "Tuberin"
}